{
  "term_label": "MutLalpha complex",
  "gene": "UniProtKB:P40692",
  "term_id": "GO:0032389",
  "gene_name": "DNA mismatch repair protein Mlh1",
  "gene_symbol": "MLH1"
}